{
  "term_label": "ATPase-coupled transmembrane transporter activity",
  "gene_symbol": "ABCA5",
  "gene": "UniProtKB:Q8WWZ7",
  "term_id": "GO:0042626",
  "gene_name": "Cholesterol transporter ABCA5"
}